regulation of respiratory burst involved in inflammatory response [GO:0060264] (biological process) Also known as: regulation of respiratory burst involved in acute inflammatory response Definition: Any process that modulates the rate, frequency or extent of a phase of elevated metabolic activity, during which oxygen consumption increases made as a defense response ; this leads to the production, by an NADH dependent system, of hydrogen peroxide (H2O2), superoxide anions and hydroxyl radicals. Sources: GOC:BHF, GOC:dph, GOC:rl, GOC:tb Subtypes: GO:0060265, negative regulation of respiratory burst involved in inflammatory response [GO:0060266] Relationships: is a type of regulation of immune effector process [GO:0002697]; is a type of regulation of innate immune response [GO:0045088]; is a type of regulation of inflammatory response [GO:0050727]; is a type of regulation of multicellular organismal process [GO:0051239]; is a type of regulation of respiratory burst [GO:0060263]; regulates respiratory burst involved in inflammatory response [GO:0002536]